acyl-[acyl-carrier-protein]-UDP-N-acetylglucosamine O-acyltransferase activity [GO:0008780] (MF) Definition: Catalysis of the reaction: a (3R)-hydroxyacyl-[ACP] + UDP-N-acetyl-alpha-D-glucosamine = a UDP-3-O-[(3R)-3-hydroxyacyl]-N-acetyl-alpha-D-glucosamine + holo-[ACP]. Sources: RHEA:67812 Relationships: is a type of O-acyltransferase activity [GO:0008374] Also known as: acyl-acyl-carrier-protein-UDP-N-acetylglucosamine O-acyltransferase, acyl-ACP-UDP-N-acetylglucosamine O-acyltransferase activity, acyl-[acyl-carrier protein]-UDP-N-acetylglucosamine O-acyltransferase activity, (R)-3-hydroxytetradecanoyl-acyl-carrier-protein:UDP-N-acetylglucosamine 3-O-(3-hydroxytetradecanoyl)transferase activity, UDP-N-acetylglucosamine acyltransferase activity, uridine diphosphoacetylglucosamine acyltransferase activity